{
  "gene_name": "Protein-tyrosine sulfotransferase 2",
  "term_id": "UNKNOWN:0002",
  "gene_symbol": "TPST2",
  "term_label": "Unknown biological process",
  "gene": "UniProtKB:O60704"
}